xylan catabolic process [GO:0045493] (biological process) Regulation: regulated by regulation of xylan catabolic process [GO:2001000]; negatively regulated by negative regulation of xylan catabolic process [GO:2001001]; positively regulated by positive regulation of xylan catabolic process [GO:2001002] Relationships: is a type of xylan metabolic process [GO:0045491]; is a type of hemicellulose catabolic process [GO:2000895] References: PMID:11931668 Sources: GOC:go_curators Subtypes: glucuronoxylan catabolic process [GO:2000886], arabinoxylan-containing compound catabolic process [GO:2000888] Also known as: xylan breakdown, xylan catabolism, xylan degradation Definition: The chemical reactions and pathways resulting in the breakdown of xylan, a polymer containing a beta-1,4-linked D-xylose backbone.